ascospore wall biogenesis [GO:0070591] (biological process) Definition: A cellular process that results in the biosynthesis of constituent macromolecules, assembly, and arrangement of constituent parts of an ascospore wall. Sources: GOC:mah Relationships: is a type of GO:0009272; is a type of spore wall biogenesis [GO:0070590]; is a type of meiotic cell cycle process [GO:1903046]; is part of GO:0030437